{
  "gene_name": "Mdm2-binding protein",
  "term_label": "traversing start control point of mitotic cell cycle",
  "gene": "UniProtKB:Q96DY7",
  "term_id": "GO:0007089",
  "gene_symbol": "MTBP"
}